{
  "gene": "UniProtKB:Q9NVN3",
  "gene_symbol": "RIC8B",
  "term_id": "GO:0005085",
  "term_label": "guanyl-nucleotide exchange factor activity",
  "gene_name": "Synembryn-B"
}